lymphoid lineage cell migration into thymus involved in thymus epithelium morphogenesis [GO:1902550] (biological process) Relationships: is a type of lymphoid lineage cell migration into thymus [GO:0097535]; is part of thymus epithelium morphogenesis [GO:0097536] References: PMID:22342843 Sources: GOC:TermGenie, GOC:cvs Definition: Any lymphoid lineage cell migration into thymus that is involved in thymus epithelium morphogenesis. Also known as: lymphoid lineage cell migration into thymus involved in thymic epithelium morphogenesis, lymphoid lineage restricted progenitor cell migration into thymus involved in thymic epithelium morphogenesis, lymphoid lineage restricted progenitor cell migration into thymus involved in thymus epithelium morphogenesis